{
  "term_label": "central nervous system development",
  "gene_symbol": "HAPLN4",
  "gene": "UniProtKB:Q86UW8",
  "term_id": "GO:0007417",
  "gene_name": "Hyaluronan and proteoglycan link protein 4"
}